{
  "term_id": "UNKNOWN:0002",
  "gene_name": "SH2 domain-containing protein 4B",
  "term_label": "Unknown biological process",
  "gene_symbol": "SH2D4B",
  "gene": "UniProtKB:Q5SQS7"
}